{
  "term_id": "GO:0005929",
  "gene": "UniProtKB:Q8N271",
  "gene_symbol": "PROM2",
  "gene_name": "Prominin-2",
  "term_label": "cilium"
}